tetrahydrofolylpolyglutamate synthase activity [GO:0004326] (molecular function) Sources: EC:6.3.2.17 Relationships: is a type of acid-amino acid ligase activity [GO:0016881]; is part of GO:0046901 Definition: Catalysis of the reaction: ATP + tetrahydrofolyl-(Glu)(n) + L-glutamate = ADP + phosphate + tetrahydrofolyl-(Glu)(n+1). Also known as: folylpolyglutamate synthase activity, FPGS activity, N(10)-formyltetrahydropteroyldiglutamate synthetase activity, N10-formyltetrahydropteroyldiglutamate synthetase activity, folate polyglutamate synthetase activity, folylpoly(gamma-glutamate) synthase activity, folylpoly-gamma-glutamate synthase activity, folylpoly-gamma-glutamate synthetase-dihydrofolate synthetase activity, folylpolyglutamate synthetase activity, folylpolyglutamyl synthetase activity, formyltetrahydropteroyldiglutamate synthetase activity, tetrahydrofolate synthase activity, tetrahydrofolate:L-glutamate gamma-ligase (ADP-forming) activity, tetrahydrofolyl-[gamma-Glu]n:L-glutamate gamma-ligase (ADP-forming), tetrahydropteroyl-[gamma-polyglutamate]:L-glutamate gamma-ligase (ADP-forming)